{
  "gene_symbol": "FCRLA",
  "term_label": "cell surface receptor signaling pathway",
  "term_id": "GO:0007166",
  "gene": "UniProtKB:Q7L513",
  "gene_name": "Fc receptor-like A"
}